positive regulation of thymocyte aggregation [GO:2000400] (biological process) Definition: Any process that activates or increases the frequency, rate or extent of thymocyte aggregation. Relationships: is a type of GO:1903039; is a type of regulation of thymocyte aggregation [GO:2000398]; positively regulates GO:0071594 Sources: GOC:BHF, GOC:mah Also known as: positive regulation of T cell precursor aggregation, positive regulation of immature T-lymphocyte aggregation, positive regulation of thymic lymphocyte aggregation, positive regulation of immature T cell aggregation, positive regulation of immature T-cell aggregation